{
  "term_label": "negative regulation of alpha-beta T cell proliferation",
  "gene_symbol": "TNFRSF14",
  "term_id": "GO:0046642",
  "gene_name": "Tumor necrosis factor receptor superfamily member 14",
  "gene": "UniProtKB:Q92956"
}